ATP-binding cassette (ABC) transporter complex [GO:0043190] (cellular component) Subtypes: ATP-binding cassette (ABC) transporter complex, transmembrane substrate-binding subunit-containing [GO:0035796], ATP-binding cassette (ABC) transporter complex, integrated substrate binding [GO:0055051], ATP-binding cassette (ABC) transporter complex, substrate-binding subunit-containing [GO:0055052], glycerol-3-phosphate-transporting ATPase complex [GO:1902517], maltose transport complex [GO:1990060], GO:1990154, GO:1990191, GO:1990193, methionine-importing ABC transporter complex [GO:1990197], GO:1990199, GO:1990222 References: PMID:11421269, PMID:15111107 Sources: GOC:jl, GOC:mtg_sensu Definition: A complex for the transport of metabolites into and out of the cell, typically comprised of four domains; two membrane-associated domains and two ATP-binding domains at the intracellular face of the membrane, that form a central pore through the plasma membrane. Each of the four core domains may be encoded as a separate polypeptide or the domains can be fused in any one of a number of ways into multidomain polypeptides. In Bacteria and Archaebacteria, ABC transporters also include substrate binding proteins to bind substrate external to the cytoplasm and deliver it to the transporter. Also known as: ABC-type efflux permease complex, ABC-type efflux porter complex, ABC-type uptake permease complex, mating pheromone exporter Relationships: is a type of ATPase dependent transmembrane transport complex [GO:0098533]; is a type of GO:0098797